{
  "term_label": "Unknown biological process",
  "term_id": "UNKNOWN:0002",
  "gene": "UniProtKB:O96001",
  "gene_name": "Protein phosphatase 1 regulatory subunit 17",
  "gene_symbol": "PPP1R17"
}